{
  "term_label": "Unknown biological process",
  "gene_symbol": "SYT16",
  "gene_name": "Synaptotagmin-16",
  "term_id": "UNKNOWN:0002",
  "gene": "UniProtKB:Q17RD7"
}